response to denervation involved in regulation of muscle adaptation [GO:0014894] (biological process) Sources: GOC:mtg_muscle Relationships: is a type of response to muscle inactivity involved in regulation of muscle adaptation [GO:0014877] Definition: Any process that results in a change in state or activity of a cell or an organism (in terms of movement, secretion, enzyme production, gene expression, etc.) as a result of a denervation stimulus. This process occurs as part of the regulation of muscle adaptation.